oncostatin M production [GO:0044808] (BP) Definition: The appearance of oncostatin M due to biosynthesis or secretion following a cellular stimulus, resulting in an increase in its intracellular or extracellular levels. Also known as: OSM production Relationships: is a type of cytokine production [GO:0001816] Sources: GOC:rv